ubiquitin-like protein conjugating enzyme activity [GO:0061650] (molecular function) Definition: Isoenergetic transfer of a ubiquitin-like protein (ULP) from one protein to another molecule, usually another protein, via the reaction X-SCP + Y = Y-SCP + X, where both the X-SCP and Y-SCP linkages are thioester bonds between the C-terminal amino acid of SCP and a sulfhydryl side group of a cysteine residue. Sources: GOC:dph Relationships: is a type of ubiquitin-like protein transferase activity [GO:0019787] Subtypes: ubiquitin conjugating enzyme activity [GO:0061631], Atg12 conjugating enzyme activity [GO:0061651], FAT10 conjugating enzyme activity [GO:0061652], ISG15 conjugating enzyme activity [GO:0061653], GO:0061654, Pup conjugating enzyme activity [GO:0061655], SUMO conjugating enzyme activity [GO:0061656], UFM1 conjugating enzyme activity [GO:0061657], GO:0061658, Atg8-family conjugating enzyme activity [GO:0141046] Also known as: E2, small conjugating protein conjugating enzyme activity